protein-N(PI)-phosphohistidine-fructose phosphotransferase system transporter activity [GO:0022877] (MF) Definition: Catalysis of the PEP-dependent, phosphoryl transfer-driven transport of substances across a membrane. The transport happens by catalysis of the reaction: protein N-phosphohistidine + fructose(out) = protein histidine + fructose phosphate(in). This differs from primary and secondary active transport in that the solute is modified during transport. Sources: GOC:mtg_transport, ISBN:0815340729 Also known as: fructose PTS transporter activity Relationships: is_a fructose transmembrane transporter activity [GO:0005353]; is_a protein-N(PI)-phosphohistidine-sugar phosphotransferase activity [GO:0008982]